{
  "gene_name": "Kin of IRRE-like protein 2",
  "gene_symbol": "KIRREL2",
  "term_id": "GO:0050839",
  "gene": "UniProtKB:Q6UWL6",
  "term_label": "cell adhesion molecule binding"
}